CXCR5 chemokine receptor binding [GO:0031724] (molecular function) Also known as: type 1 Burkitt's lymphoma receptor binding, CXCR5 chemokine receptor ligand Definition: Binding to a CXCR5 chemokine receptor. Relationships: is a type of CXCR chemokine receptor binding [GO:0045236] Sources: GOC:mah, GOC:nln